{
  "gene_name": "Endoribonuclease Dicer",
  "gene_symbol": "DICER1",
  "term_label": "cytoplasm",
  "term_id": "GO:0005737",
  "gene": "UniProtKB:Q9UPY3"
}